{
  "term_id": "GO:0017147",
  "gene_symbol": "ROR2",
  "gene": "UniProtKB:Q01974",
  "term_label": "Wnt-protein binding",
  "gene_name": "Tyrosine-protein kinase transmembrane receptor ROR2"
}